{
  "term_label": "Unknown molecular function",
  "gene_name": "Transmembrane protein 170A",
  "term_id": "UNKNOWN:0001",
  "gene": "UniProtKB:Q8WVE7",
  "gene_symbol": "TMEM170A"
}